{
  "gene_symbol": "RSPH1",
  "gene_name": "Radial spoke head 1 homolog",
  "gene": "UniProtKB:Q8WYR4",
  "term_label": "spermatid development",
  "term_id": "GO:0007286"
}